{
  "gene_symbol": "G6PC3",
  "gene": "UniProtKB:Q9BUM1",
  "term_label": "glucose 6-phosphate metabolic process",
  "term_id": "GO:0051156",
  "gene_name": "Glucose-6-phosphatase 3"
}